{
  "gene_symbol": "KCTD14",
  "term_label": "Unknown molecular function",
  "gene_name": "BTB_POZ domain-containing protein KCTD14",
  "gene": "UniProtKB:Q9BQ13",
  "term_id": "UNKNOWN:0001"
}